{
  "gene": "UniProtKB:Q9UNK0",
  "gene_symbol": "STX8",
  "term_label": "vesicle fusion",
  "term_id": "GO:0006906",
  "gene_name": "Syntaxin-8"
}